{
  "term_id": "GO:0004725",
  "term_label": "protein tyrosine phosphatase activity",
  "gene_symbol": "EYA3",
  "gene_name": "Eyes absent homolog 3",
  "gene": "UniProtKB:Q99504"
}